{
  "term_id": "GO:0098609",
  "gene_name": "Desmocollin-2",
  "gene": "UniProtKB:Q02487",
  "term_label": "cell-cell adhesion",
  "gene_symbol": "DSC2"
}